{
  "term_id": "GO:0030674",
  "term_label": "protein-macromolecule adaptor activity",
  "gene": "UniProtKB:Q9H4M9",
  "gene_symbol": "EHD1",
  "gene_name": "EH domain-containing protein 1"
}